regulation of osteoclast proliferation [GO:0090289] (biological process) Subtypes: positive regulation of osteoclast proliferation [GO:0090290], negative regulation of osteoclast proliferation [GO:0090291] Relationships: is a type of regulation of leukocyte proliferation [GO:0070663]; regulates osteoclast proliferation [GO:0002158] Sources: GOC:tb Definition: Any process that modulates the rate, frequency, or extent of the multiplication or reproduction of osteoclasts, resulting in the expansion of an osteoclast cell population.